{
  "gene": "UniProtKB:Q71F23",
  "term_label": "Unknown molecular function",
  "gene_symbol": "CENPU",
  "term_id": "UNKNOWN:0001",
  "gene_name": "Centromere protein U"
}